vitamin D3 metabolic process [GO:0070640] (biological process) Subtypes: calcitriol biosynthetic process from calciol [GO:0036378], vitamin D3 catabolic process [GO:1901754], vitamin D3 biosynthetic process [GO:1901755] Relationships: is a type of vitamin D metabolic process [GO:0042359]; is a type of secondary alcohol metabolic process [GO:1902652] Also known as: calciol metabolic process, cholecalciferol metabolic process, vitamin D3 metabolism Sources: GOC:BHF, GOC:mah Definition: The chemical reactions and pathways involving vitamin D3, (3S,5Z,7E)-9,10-secocholesta-5,7,10(19)-trien-3-ol.